{
  "gene_name": "F-box_LRR-repeat protein 7",
  "term_id": "UNKNOWN:0001",
  "gene": "UniProtKB:Q9UJT9",
  "term_label": "Unknown molecular function",
  "gene_symbol": "FBXL7"
}